regulation of methane biosynthetic process from carbon monoxide [GO:1900336] (biological process) Definition: Any process that modulates the frequency, rate or extent of methane biosynthetic process from carbon monoxide. Subtypes: negative regulation of methane biosynthetic process from carbon monoxide [GO:1900337], positive regulation of methane biosynthetic process from carbon monoxide [GO:1900338] Relationships: is a type of GO:0043457; is a type of GO:1901577; regulates GO:2001134 Sources: GOC:TermGenie, GOC:mengo_curators